D-threonine aldolase activity [GO:0043876] (molecular function) References: PMID:9642221 Sources: MetaCyc:4.1.2.42-RXN Relationships: is a type of GO:0016832 Definition: Catalysis of the reaction: D-threonine (or D-allo-threonine) = glycine + acetaldehyde. Also known as: D-TA, D-allo-TA, D-allo-threonine aldolase activity, low-specificity D-threonine aldolase, DtaAS